{
  "gene_symbol": "SGSM2",
  "gene_name": "Small G protein signaling modulator 2",
  "term_id": "UNKNOWN:0002",
  "term_label": "Unknown biological process",
  "gene": "UniProtKB:O43147"
}